{
  "gene_symbol": "STX1A",
  "term_id": "GO:0048278",
  "term_label": "vesicle docking",
  "gene": "UniProtKB:Q16623",
  "gene_name": "Syntaxin-1A"
}